positive regulation of adherens junction organization [GO:1903393] (BP) Definition: Any process that activates or increases the frequency, rate or extent of adherens junction organization. References: PMID:21724833 Sources: GOC:TermGenie, GOC:als, GO_REF:0000058 Also known as: positive regulation of adherens junction assembly and maintenance, positive regulation of adherens junction organisation, up regulation of adherens junction assembly and maintenance, up regulation of adherens junction organisation, up regulation of adherens junction organization, up-regulation of adherens junction assembly and maintenance, up-regulation of adherens junction organisation, up-regulation of adherens junction organization, upregulation of adherens junction assembly and maintenance, upregulation of adherens junction organisation, upregulation of adherens junction organization, activation of adherens junction assembly and maintenance, activation of adherens junction organisation, activation of adherens junction organization Relationships: is_a GO:0051130; is a type of regulation of adherens junction organization [GO:1903391]; positively regulates adherens junction organization [GO:0034332]